TCR signalosome [GO:0036398] (cellular component) Definition: A multi-protein complex containing at least the T-cell receptor complex and the LAT (linker for activation of T cells) scaffold protein. Also contains a variety of signaling proteins including co-receptors, kinases, phosphatases and adaptors such as CD8. Connects events on the plasma membrane to distal signaling cascades to ultimately modulate T cell biology. Relationships: is a type of GO:0032991; has part T cell receptor complex [GO:0042101] Also known as: LAT signalosome, linker for activation of T cells signalosome References: PMID:17534068, PMID:20107804, PMID:22426112 Sources: GOC:krc